{
  "gene_symbol": "Q6ZRU5",
  "gene": "UniProtKB:Q6ZRU5",
  "term_id": "UNKNOWN:0003",
  "gene_name": "Putative uncharacterized protein FLJ46089",
  "term_label": "Unknown cellular component"
}